gated channel activity [GO:0022836] (molecular function) Sources: GOC:mtg_transport Subtypes: mechanosensitive monoatomic ion channel activity [GO:0008381], voltage-gated channel activity [GO:0022832], ligand-gated channel activity [GO:0022834], GO:0097603, G-protein gated monoatomic ion channel activity [GO:0099099], osmolarity-sensing monoatomic cation channel activity [GO:1990760] Relationships: is a type of channel activity [GO:0015267] Definition: Enables the transmembrane transfer of a solute by a channel that opens in response to a specific stimulus.